{
  "term_id": "GO:0003924",
  "gene": "UniProtKB:Q5HYI8",
  "gene_symbol": "RABL3",
  "term_label": "GTPase activity",
  "gene_name": "Rab-like protein 3"
}